{
  "gene": "UniProtKB:P04196",
  "term_id": "GO:0051918",
  "term_label": "negative regulation of fibrinolysis",
  "gene_name": "Histidine-rich glycoprotein",
  "gene_symbol": "HRG"
}